{
  "term_label": "deoxycytidine kinase activity",
  "gene_name": "Deoxycytidine kinase",
  "gene": "UniProtKB:P27707",
  "gene_symbol": "DCK",
  "term_id": "GO:0004137"
}